bis(5'-nucleosidyl) oligophosphate catabolic process [GO:0015958] (biological process) References: PMID:10970777 Sources: GOC:mah Definition: The chemical reactions and pathways resulting in the breakdown of a bis(5'-nucleosidyl) oligophosphate, a compound formed of two nucleosides joined together through their 5' carbons by a chain of phosphate molecules. Also known as: bis(5'-nucleosidyl) oligophosphate breakdown, bis(5'-nucleosidyl) oligophosphate catabolism, bis(5'-nucleosidyl) oligophosphate degradation Relationships: is_a nucleotide catabolic process [GO:0009166]